{
  "gene_name": "Elongin-C",
  "gene_symbol": "ELOC",
  "term_id": "GO:0006511",
  "gene": "UniProtKB:Q15369",
  "term_label": "ubiquitin-dependent protein catabolic process"
}